{
  "term_id": "GO:0007165",
  "term_label": "signal transduction",
  "gene_name": "Serine_threonine-protein kinase VRK1",
  "gene": "UniProtKB:Q99986",
  "gene_symbol": "VRK1"
}